embryonic neurocranium morphogenesis [GO:0048702] (biological process) References: PMID:16049113 Sources: GOC:dsf, GOC:jid Relationships: is a type of embryonic morphogenesis [GO:0048598]; BFO_0000050 embryonic cranial skeleton morphogenesis [GO:0048701] Also known as: embryonic braincase morphogenesis, embryonic chondrocranium morphogenesis Definition: The process in which the anatomical structures of the neurocranium are generated and organized during the embryonic phase. The neurocranium is the portion of the vertebrate skull surrounding the brain.